negative regulation of humoral immune response mediated by circulating immunoglobulin [GO:0002924] (biological process) Definition: Any process that stops, prevents, or reduces the frequency, rate, or extent of a humoral immune response mediated by circulating immunoglobulin. Subtypes: negative regulation of complement activation, classical pathway [GO:0045959] Also known as: down regulation of humoral immune response mediated by circulating immunoglobulin, down-regulation of humoral immune response mediated by circulating immunoglobulin, downregulation of humoral immune response mediated by circulating immunoglobulin, inhibition of humoral immune response mediated by circulating immunoglobulin Sources: GOC:add Relationships: is a type of negative regulation of immunoglobulin mediated immune response [GO:0002890]; is a type of negative regulation of humoral immune response [GO:0002921]; is a type of regulation of humoral immune response mediated by circulating immunoglobulin [GO:0002923]; negatively regulates humoral immune response mediated by circulating immunoglobulin [GO:0002455]